{
  "term_id": "GO:0004687",
  "term_label": "myosin light chain kinase activity",
  "gene_name": "Myosin light chain kinase 3",
  "gene": "UniProtKB:Q32MK0",
  "gene_symbol": "MYLK3"
}